{
  "term_id": "GO:0006686",
  "gene_name": "Phosphatidylcholine:ceramide cholinephosphotransferase 1",
  "gene_symbol": "SGMS1",
  "gene": "UniProtKB:Q86VZ5",
  "term_label": "sphingomyelin biosynthetic process"
}